{
  "term_label": "Unknown biological process",
  "gene_name": "Alpha-centractin",
  "term_id": "UNKNOWN:0002",
  "gene": "UniProtKB:P61163",
  "gene_symbol": "ACTR1A"
}